{
  "gene": "UniProtKB:P50222",
  "term_label": "somite development",
  "gene_symbol": "MEOX2",
  "gene_name": "Homeobox protein MOX-2",
  "term_id": "GO:0061053"
}